{
  "term_label": "Unknown cellular component",
  "term_id": "UNKNOWN:0003",
  "gene": "UniProtKB:Q674X7",
  "gene_name": "Kazrin",
  "gene_symbol": "KAZN"
}